rhombomere 5 formation [GO:0021666] (biological process) Definition: The process that gives rise to rhombomere 5. This process pertains to the initial formation of a structure from unspecified parts. Rhombomeres are transverse segments of the developing rhombencephalon. Rhombomeres are lineage restricted, express different genes from one another, and adopt different developmental fates. Rhombomeres are numbered in anterior to posterior order. Relationships: is a type of GO:0021594; is part of rhombomere 5 morphogenesis [GO:0021664] Sources: GOC:cls, GOC:curators, GOC:dgh, GOC:dph, GOC:jid